{
  "term_id": "UNKNOWN:0001",
  "gene_name": "Centrosomal protein of 104 kDa",
  "gene_symbol": "CEP104",
  "gene": "UniProtKB:O60308",
  "term_label": "Unknown molecular function"
}